cell tip growth [GO:0009932] (BP) Definition: Growth that occurs specifically at the tip of a cell. Sources: GOC:jid Relationships: is_a GO:0009826 Subtypes: pollen tube growth [GO:0009860], root hair cell tip growth [GO:0048768]